{
  "term_label": "Unknown biological process",
  "term_id": "UNKNOWN:0002",
  "gene": "UniProtKB:Q6AWC8",
  "gene_symbol": "Q6AWC8",
  "gene_name": "Putative uncharacterized protein LOC100129027"
}